{
  "gene_name": "Interferon alpha-5",
  "term_id": "GO:0005132",
  "gene_symbol": "IFNA5",
  "term_label": "type I interferon receptor binding",
  "gene": "UniProtKB:P01569"
}